{
  "gene_name": "Oocyte-secreted protein 3",
  "term_label": "Unknown cellular component",
  "term_id": "UNKNOWN:0003",
  "gene": "UniProtKB:A0A2R8YFM6",
  "gene_symbol": "OOSP3"
}